{
  "term_id": "GO:0044539",
  "term_label": "long-chain fatty acid import into cell",
  "gene_symbol": "SLC27A5",
  "gene": "UniProtKB:Q9Y2P5",
  "gene_name": "Long-chain fatty acid transport protein 5"
}